{
  "term_id": "GO:0046839",
  "gene_name": "Phospholipid phosphatase-related protein type 3",
  "term_label": "phospholipid dephosphorylation",
  "gene_symbol": "PLPPR3",
  "gene": "UniProtKB:Q6T4P5"
}